{
  "gene": "UniProtKB:Q3L8U1",
  "gene_name": "Chromodomain-helicase-DNA-binding protein 9",
  "term_label": "Unknown cellular component",
  "gene_symbol": "CHD9",
  "term_id": "UNKNOWN:0003"
}